{
  "gene_name": "G-protein-signaling modulator 2",
  "term_label": "establishment of mitotic spindle orientation",
  "gene": "UniProtKB:P81274",
  "term_id": "GO:0000132",
  "gene_symbol": "GPSM2"
}